{
  "gene": "UniProtKB:Q92485",
  "gene_name": "Acid sphingomyelinase-like phosphodiesterase 3b",
  "gene_symbol": "SMPDL3B",
  "term_id": "GO:0008081",
  "term_label": "phosphoric diester hydrolase activity"
}